{
  "gene_symbol": "ASB11",
  "term_label": "Unknown molecular function",
  "gene": "UniProtKB:Q8WXH4",
  "term_id": "UNKNOWN:0001",
  "gene_name": "Ankyrin repeat and SOCS box protein 11"
}